{
  "gene_symbol": "SOCS1",
  "term_label": "cytokine-mediated signaling pathway",
  "gene": "UniProtKB:O15524",
  "term_id": "GO:0019221",
  "gene_name": "Suppressor of cytokine signaling 1"
}